{
  "term_id": "GO:0016529",
  "gene_symbol": "PLN",
  "gene_name": "Cardiac phospholamban",
  "term_label": "sarcoplasmic reticulum",
  "gene": "UniProtKB:P26678"
}